2-oxo-delta3-4,5,5-trimethylcyclopentenylacetyl-CoA synthetase activity [GO:0018855] (molecular function) Sources: UM-BBD_reactionID:r0429 Relationships: is a type of GO:0016405; is a type of acid-thiol ligase activity [GO:0016878] Definition: Catalysis of the reaction: 2-oxo-delta3-4,5,5-trimethylcyclopentenylacetate + ATP + CoA = AMP + diphosphate + 2-oxo-delta3-4,5,5-trimethylcyclopentenylacetyl-CoA.